nucleoside triphosphate biosynthetic process [GO:0009142] (biological process) Relationships: is a type of GO:0009141; is_a nucleoside phosphate biosynthetic process [GO:1901293] Sources: GOC:go_curators, ISBN:0198506732 Also known as: nucleoside triphosphate anabolism, nucleoside triphosphate biosynthesis, nucleoside triphosphate formation, nucleoside triphosphate synthesis Definition: The chemical reactions and pathways resulting in the formation of a nucleoside triphosphate, a compound consisting of a nucleobase linked to a deoxyribose or ribose sugar esterified with triphosphate on the sugar. Subtypes: purine nucleoside triphosphate biosynthetic process [GO:0009145], GO:0009148, GO:0009201, GO:0009202